{
  "term_id": "UNKNOWN:0003",
  "gene": "UniProtKB:A0A0B4J1V7",
  "gene_name": "Probable non-functional immunoglobulin heavy variable 7-81",
  "term_label": "Unknown cellular component",
  "gene_symbol": "IGHV7-81"
}